kynurenine 3-monooxygenase activity [GO:0004502] (molecular function) Sources: EC:1.14.13.9, RHEA:20545 Relationships: is a type of oxidoreductase activity, acting on paired donors, with incorporation or reduction of molecular oxygen, NAD(P)H as one donor, and incorporation of one atom of oxygen [GO:0016709] Also known as: kynurenine 3-hydroxylase activity, L-kynurenine,NADPH:oxygen oxidoreductase (3-hydroxylating), L-kynurenine-3-hydroxylase activity, kynurenine hydroxylase activity Definition: Catalysis of the reaction: L-kynurenine + H+ + NADPH + O2 = 3-hydroxy-L-kynurenine + H2O + NADP+.